{
  "term_id": "GO:0015375",
  "term_label": "glycine:sodium symporter activity",
  "gene_name": "Sodium- and chloride-dependent glycine transporter 2",
  "gene_symbol": "SLC6A5",
  "gene": "UniProtKB:Q9Y345"
}